regulation of chemokine-mediated signaling pathway [GO:0070099] (biological process) Sources: GOC:mah Definition: Any process that modulates the rate, frequency or extent of a chemokine-mediated signaling pathway. Relationships: is a type of regulation of cytokine-mediated signaling pathway [GO:0001959]; is a type of GO:0008277; regulates GO:0070098 Also known as: regulation of chemokine-mediated signalling pathway Subtypes: negative regulation of chemokine-mediated signaling pathway [GO:0070100], positive regulation of chemokine-mediated signaling pathway [GO:0070101], GO:1903080